{
  "gene_symbol": "SHQ1",
  "gene": "UniProtKB:Q6PI26",
  "gene_name": "Protein SHQ1 homolog",
  "term_label": "cytoplasm",
  "term_id": "GO:0005737"
}